{
  "gene": "UniProtKB:Q9HAZ1",
  "gene_symbol": "CLK4",
  "term_id": "GO:0005634",
  "gene_name": "Dual specificity protein kinase CLK4",
  "term_label": "nucleus"
}